{
  "gene_symbol": "IGF2BP3",
  "term_id": "GO:0007399",
  "gene": "UniProtKB:O00425",
  "term_label": "nervous system development",
  "gene_name": "Insulin-like growth factor 2 mRNA-binding protein 3"
}